{
  "gene": "UniProtKB:Q4VXF1",
  "gene_symbol": "FAM74A3",
  "gene_name": "Putative protein FAM74A3",
  "term_label": "Unknown biological process",
  "term_id": "UNKNOWN:0002"
}